acyltransferase activity [GO:0016746] (molecular function) Relationships: is a type of GO:0016740 Definition: Catalysis of the transfer of an acyl group from one compound (donor) to another (acceptor). Sources: EC:2.3.-.- Subtypes: GO:0016747, aminoacyltransferase activity [GO:0016755], acyltransferase activity, acyl groups converted into alkyl on transfer [GO:0046912] Also known as: transferase activity, transferring acyl groups